P granule assembly [GO:1903863] (BP) References: PMID:25535836 Sources: GOC:TermGenie, GOC:kmv, GO_REF:0000079 Relationships: is a type of P granule organization [GO:0030719]; is a type of GO:0140694 Definition: The aggregation, arrangement and bonding together of a set of components to form a P granule. Also known as: P granule formation, germline granule assembly, germline granule formation, polar granule assembly, polar granule formation